protein denaturation [GO:0030164] (biological process) Relationships: is a type of protein catabolic process [GO:0030163] Definition: Structural change in proteins which destroys the native, active configuration without rupture of peptide bonds. Sources: GOC:kd, ISBN:3110145359